{
  "term_label": "endosome membrane",
  "gene": "UniProtKB:Q5VST6",
  "term_id": "GO:0010008",
  "gene_name": "Alpha_beta hydrolase domain-containing protein 17B",
  "gene_symbol": "ABHD17B"
}